{
  "gene": "UniProtKB:Q15399",
  "gene_name": "Toll-like receptor 1",
  "term_id": "GO:0006954",
  "gene_symbol": "TLR1",
  "term_label": "inflammatory response"
}